{
  "term_label": "microtubule polymerization",
  "gene": "UniProtKB:P59282",
  "term_id": "GO:0046785",
  "gene_symbol": "TPPP2",
  "gene_name": "Tubulin polymerization-promoting protein family member 2"
}